novobiocin biosynthetic process [GO:0043642] (biological process) Sources: GOC:jl Definition: The chemical reactions and pathways resulting in the formation of novobiocin, a coumarin antibiotic produced by the bacterium Gyrasestreptomyces spheroides, that acts by inhibiting DNA gyrase. Relationships: is a type of coumarin biosynthetic process [GO:0009805]; is a type of glycoside biosynthetic process [GO:0016138]; is a type of GO:0017000; is a type of amide biosynthetic process [GO:0043604]; is a type of phenol-containing compound biosynthetic process [GO:0046189]; is a type of ether biosynthetic process [GO:1901503]